{
  "term_label": "regulation of membrane lipid distribution",
  "gene": "UniProtKB:A6NGC4",
  "term_id": "GO:0097035",
  "gene_name": "TLC domain-containing protein 2",
  "gene_symbol": "TLCD2"
}